regulation of blood vessel remodeling [GO:0060312] (biological process) Relationships: is a type of GO:0022603; is_a regulation of tissue remodeling [GO:0034103]; regulates blood vessel remodeling [GO:0001974] Subtypes: negative regulation of blood vessel remodeling [GO:0060313], regulation of pulmonary blood vessel remodeling [GO:1905109], GO:2000504 Also known as: regulation of blood vessel remodelling Sources: GOC:BHF, GOC:dph, GOC:tb Definition: Any process that modulates the rate, frequency or extent of blood vessel remodeling, the reorganization or renovation of existing blood vessels.